{
  "term_id": "GO:0070328",
  "gene_name": "Cholesteryl ester transfer protein",
  "gene_symbol": "CETP",
  "gene": "UniProtKB:P11597",
  "term_label": "triglyceride homeostasis"
}